{
  "gene_name": "Mediator of RNA polymerase II transcription subunit 9",
  "gene": "UniProtKB:Q9NWA0",
  "term_id": "UNKNOWN:0002",
  "term_label": "Unknown biological process",
  "gene_symbol": "MED9"
}